{
  "term_label": "Unknown cellular component",
  "gene": "UniProtKB:Q9HBF5",
  "gene_name": "Suppressor of tumorigenicity 20 protein",
  "term_id": "UNKNOWN:0003",
  "gene_symbol": "ST20"
}